protein localization to euchromatin [GO:1905632] (biological process) References: PMID:20889714 Sources: GOC:TermGenie, GO_REF:0000087 Definition: A process in which a protein is transported to, or maintained in, a location within an euchromatin. Relationships: is a type of protein localization to chromatin [GO:0071168] Also known as: protein localisation in euchromatin, protein localisation to euchromatin, protein localization in euchromatin